{
  "term_label": "extracellular space",
  "gene": "UniProtKB:Q8TDE3",
  "gene_symbol": "RNASE8",
  "term_id": "GO:0005615",
  "gene_name": "Ribonuclease 8"
}